{
  "term_id": "GO:0006357",
  "gene_name": "Nuclear receptor subfamily 5 group A member 2",
  "term_label": "regulation of transcription by RNA polymerase II",
  "gene": "UniProtKB:O00482",
  "gene_symbol": "NR5A2"
}